monoatomic cation efflux transmembrane transporter activity [GO:0046583] (molecular function) Sources: GOC:ai, GOC:mtg_transport, ISBN:0815340729 Also known as: cation efflux transmembrane transporter activity, cation efflux permease activity Relationships: is_a monoatomic cation transmembrane transporter activity [GO:0008324]; is a type of efflux transmembrane transporter activity [GO:0015562] Definition: Enables the transfer of a cation or cations from the inside of the cell to the outside of the cell across a membrane. Subtypes: zinc efflux transmembrane transporter activity [GO:0022883]